{
  "gene_symbol": "PRAM1",
  "term_label": "plasma membrane",
  "term_id": "GO:0005886",
  "gene": "UniProtKB:Q96QH2",
  "gene_name": "PML-RARA-regulated adapter molecule 1"
}